{
  "term_label": "membrane",
  "gene_symbol": "TMEM151B",
  "term_id": "GO:0016020",
  "gene_name": "Transmembrane protein 151B",
  "gene": "UniProtKB:Q8IW70"
}